myotome development [GO:0061055] (biological process) Regulation: positively regulated by positive regulation of myotome development [GO:2000287]; regulated by regulation of myotome development [GO:2000290] Relationships: is a type of GO:0048856; BFO_0000050 somite development [GO:0061053] Sources: GOC:dph Definition: The progression of the myotome over time, from its formation to the mature structure. The myotome is the portion of the somite that will give rise to muscle.